{
  "term_id": "GO:0005737",
  "gene_name": "Homeodomain-interacting protein kinase 4",
  "gene": "UniProtKB:Q8NE63",
  "gene_symbol": "HIPK4",
  "term_label": "cytoplasm"
}